{
  "gene_symbol": "NLRP2B",
  "term_id": "UNKNOWN:0003",
  "term_label": "Unknown cellular component",
  "gene_name": "NLR family pyrin domain-containing protein 2B",
  "gene": "UniProtKB:P0DMW2"
}